(17Z)-protosta-17(20),24-dien-3beta-ol biosynthetic process [GO:1900581] (biological process) Definition: The chemical reactions and pathways resulting in the formation of (17Z)-protosta-17(20),24-dien-3beta-ol. Sources: GOC:TermGenie, GOC:di Relationships: is_a steroid biosynthetic process [GO:0006694]; is a type of GO:0010686; is_a secondary metabolite biosynthetic process [GO:0044550]; is_a secondary alcohol biosynthetic process [GO:1902653] Also known as: (17Z)-protosta-17(20),24-dien-3beta-ol anabolism, (17Z)-protosta-17(20),24-dien-3beta-ol biosynthesis, (17Z)-protosta-17(20),24-dien-3beta-ol formation, (17Z)-protosta-17(20),24-dien-3beta-ol synthesis